{
  "term_label": "chemoattractant activity",
  "gene": "UniProtKB:P49767",
  "gene_name": "Vascular endothelial growth factor C",
  "gene_symbol": "VEGFC",
  "term_id": "GO:0042056"
}